{
  "gene_symbol": "CPSF3",
  "gene_name": "Cleavage and polyadenylation specificity factor subunit 3",
  "term_label": "mRNA cleavage and polyadenylation specificity factor complex",
  "term_id": "GO:0005847",
  "gene": "UniProtKB:Q9UKF6"
}